left caudal flagellum [GO:0097560] (cellular component) Also known as: left caudal cilium Relationships: is a type of 9+2 motile cilium [GO:0097729] Note: Note that we deem cilium and microtubule-based flagellum to be equivalent; the primary term name reflects frequency of use. Also note that, due to the asymmetric nature of the Giardia trophozoite, this term is defined spatially as the trophozoite is viewed from the dorsal side, with the two nuclei dorsal to the ventral disc, and the ventral disc toward the anterior. References: PMID:16607022, PMID:5961344 Sources: GOC:giardia, ISBN:9780124260207 Definition: A cilium (also called flagellum) found in Giardia species (trophozoite stage). It is nucleated by the left caudal basal body, extending cytoplasmically and exiting at the posterior end of the cell body.